{
  "gene_symbol": "SCN1B",
  "gene": "UniProtKB:Q07699",
  "gene_name": "Sodium channel subunit beta-1",
  "term_id": "GO:0001518",
  "term_label": "voltage-gated sodium channel complex"
}